{
  "gene_name": "6-pyruvoyl tetrahydrobiopterin synthase",
  "term_id": "GO:0003874",
  "gene_symbol": "PTS",
  "term_label": "6-pyruvoyltetrahydropterin synthase activity",
  "gene": "UniProtKB:Q03393"
}